{
  "gene": "UniProtKB:Q9H3M0",
  "term_label": "action potential",
  "gene_symbol": "KCNF1",
  "term_id": "GO:0001508",
  "gene_name": "Potassium voltage-gated channel subfamily F member 1"
}